{
  "gene_symbol": "PRX",
  "term_label": "nucleus",
  "gene_name": "Periaxin",
  "gene": "UniProtKB:Q9BXM0",
  "term_id": "GO:0005634"
}